{
  "term_id": "GO:0005261",
  "gene": "UniProtKB:Q8IU99",
  "term_label": "monoatomic cation channel activity",
  "gene_symbol": "CALHM1",
  "gene_name": "Calcium homeostasis modulator protein 1"
}